calcium channel complex [GO:0034704] (cellular component) Definition: An ion channel complex through which calcium ions pass. Sources: GOC:mah Relationships: is a type of cation channel complex [GO:0034703] Subtypes: voltage-gated calcium channel complex [GO:0005891], GO:1990246